{
  "term_id": "UNKNOWN:0003",
  "term_label": "Unknown cellular component",
  "gene": "UniProtKB:Q06210",
  "gene_name": "Glutamine--fructose-6-phosphate aminotransferase [isomerizing] 1",
  "gene_symbol": "GFPT1"
}